{
  "term_id": "GO:0005634",
  "gene_symbol": "LHX2",
  "gene": "UniProtKB:P50458",
  "gene_name": "LIM_homeobox protein Lhx2",
  "term_label": "nucleus"
}